{
  "gene_name": "Nephrocystin-4",
  "term_id": "GO:0090090",
  "gene": "UniProtKB:O75161",
  "term_label": "negative regulation of canonical Wnt signaling pathway",
  "gene_symbol": "NPHP4"
}